activating MHC class Ib receptor activity [GO:0062081] (molecular function) Sources: DOI:10.1002/9780470015902.a0024246 Definition: Combining with a MHC class Ib protein complex to mediate signaling that activates a lymphocyte. Relationships: is a type of MHC class Ib receptor activity [GO:0032394]